cytoplasmic replication fork [GO:0043597] (cellular component) Relationships: is a type of replication fork [GO:0005657]; is part of cytoplasm [GO:0005737] Sources: GOC:jl, GOC:mtg_sensu Definition: The Y-shaped region of a cytoplasmic replicating DNA molecule, resulting from the separation of the DNA strands and in which the synthesis of new strands takes place. Also includes associated protein complexes.